ovarian follicle rupture [GO:0001543] (biological process) Definition: Disruption of theca cell layer releasing follicular fluid and/or the oocyte. Sources: https://www.ncbi.nlm.nih.gov/books/NBK279054/ Relationships: is a type of ovulation cycle process [GO:0022602]; is part of ovulation from ovarian follicle [GO:0001542]